{
  "term_id": "GO:0001520",
  "gene_name": "Outer dense fiber protein 1",
  "term_label": "outer dense fiber",
  "gene_symbol": "ODF1",
  "gene": "UniProtKB:Q14990"
}